mammillary axonal complex development [GO:0061373] (biological process) Definition: The progression of the mammillary axonal complex over time, from its formation to the mature structure. The mammillary axonal complex is formed by the axons from the lateral, medial mammillary and the dorsal premammillary nuclei which share a branching pattern. Every neuron gives off one axonal stem that bifurcates into 2 branches. One of the branches is directed dorsally to the thalamus and another caudally to the midbrain. Relationships: is a type of GO:0048856; BFO_0000050 GO:0021767 References: PMID:10662642 Sources: GOC:dph, GOC:yaf